{
  "term_id": "GO:0006004",
  "gene_symbol": "FUCA2",
  "term_label": "fucose metabolic process",
  "gene_name": "Plasma alpha-L-fucosidase",
  "gene": "UniProtKB:Q9BTY2"
}